{
  "term_label": "Unknown cellular component",
  "gene": "UniProtKB:Q96AQ1",
  "gene_symbol": "CCDC74A",
  "term_id": "UNKNOWN:0003",
  "gene_name": "Coiled-coil domain-containing protein 74A"
}